positive regulation of tight junction disassembly [GO:1905075] (biological process) Definition: Any process that activates or increases the frequency, rate or extent of tight junction disassembly. References: PMID:18718461 Sources: GOC:BHF, GOC:TermGenie, GOC:rl, GO_REF:0000058 Relationships: is a type of GO:0051130; is a type of regulation of tight junction disassembly [GO:1905073]; positively regulates tight junction disassembly [GO:1905071] Also known as: positive regulation of occluding cell junction disassembly, positive regulation of occluding junction disassembly, up regulation of occluding cell junction disassembly, up regulation of tight junction disassembly, up-regulation of occluding cell junction disassembly, up-regulation of tight junction disassembly, upregulation of occluding cell junction disassembly, upregulation of tight junction disassembly, activation of occluding cell junction disassembly, activation of occluding junction disassembly, activation of tight junction disassembly